{
  "term_id": "GO:0005251",
  "gene_symbol": "KCNC3",
  "gene": "UniProtKB:Q14003",
  "term_label": "delayed rectifier potassium channel activity",
  "gene_name": "Potassium voltage-gated channel subfamily C member 3"
}